{
  "term_id": "GO:0003713",
  "gene": "UniProtKB:Q93074",
  "gene_name": "Mediator of RNA polymerase II transcription subunit 12",
  "gene_symbol": "MED12",
  "term_label": "transcription coactivator activity"
}